{
  "term_label": "Unknown biological process",
  "gene_symbol": "MFSD11",
  "gene_name": "UNC93-like protein MFSD11",
  "term_id": "UNKNOWN:0002",
  "gene": "UniProtKB:O43934"
}